chloride:monoatomic cation symporter activity [GO:0015377] (molecular function) Also known as: cation:chloride cotransporter activity, cation:chloride symporter activity Subtypes: sodium:chloride symporter activity [GO:0015378], GO:0015379 Definition: Enables the transfer of a solute or solutes from one side of a membrane to the other according to the reaction: cation(out) + Cl-(out) = cation(in) + Cl-(in). References: PMID:31747317 Relationships: is a type of GO:0015108; is a type of GO:0015296